{
  "term_label": "Unknown cellular component",
  "term_id": "UNKNOWN:0003",
  "gene": "UniProtKB:Q86X02",
  "gene_name": "Cerebellar degeneration-related protein 2-like",
  "gene_symbol": "CDR2L"
}